{
  "gene": "UniProtKB:A0A1W2PR82",
  "gene_name": "Protein PERCC1",
  "term_label": "Unknown cellular component",
  "term_id": "UNKNOWN:0003",
  "gene_symbol": "PERCC1"
}